{
  "term_id": "GO:0051604",
  "gene_name": "Granzyme M",
  "gene": "UniProtKB:P51124",
  "gene_symbol": "GZMM",
  "term_label": "protein maturation"
}